{
  "gene_name": "Uncharacterized protein C10orf55",
  "gene_symbol": "C10orf55",
  "term_label": "Unknown cellular component",
  "gene": "UniProtKB:Q5SWW7",
  "term_id": "UNKNOWN:0003"
}